{
  "term_label": "plasma membrane",
  "gene": "UniProtKB:Q6ZWK6",
  "gene_symbol": "TMPRSS11F",
  "gene_name": "Transmembrane protease serine 11F",
  "term_id": "GO:0005886"
}